negative regulation of vascular associated smooth muscle cell migration [GO:1904753] (biological process) Also known as: down regulation of vascular associated smooth muscle cell migration, down regulation of vascular smooth muscle cell migration, down-regulation of vascular associated smooth muscle cell migration, down-regulation of vascular smooth muscle cell migration, downregulation of vascular associated smooth muscle cell migration, downregulation of vascular smooth muscle cell migration, negative regulation of vascular smooth muscle cell migration, inhibition of vascular associated smooth muscle cell migration, inhibition of vascular smooth muscle cell migration Relationships: is a type of negative regulation of smooth muscle cell migration [GO:0014912]; is a type of GO:1904752; negatively regulates vascular associated smooth muscle cell migration [GO:1904738] References: PMID:20693317 Sources: GOC:BHF, GOC:BHF_miRNA, GOC:TermGenie, GOC:rph, GO_REF:0000058 Definition: Any process that stops, prevents or reduces the frequency, rate or extent of vascular associated smooth muscle cell migration.